{
  "gene": "UniProtKB:P55040",
  "term_label": "plasma membrane",
  "term_id": "GO:0005886",
  "gene_symbol": "GEM",
  "gene_name": "GTP-binding protein GEM"
}